{
  "gene_name": "Transmembrane inner ear expressed protein",
  "gene": "UniProtKB:Q8NEW7",
  "term_label": "Unknown molecular function",
  "gene_symbol": "TMIE",
  "term_id": "UNKNOWN:0001"
}